trans-aconitate 3-methyltransferase activity [GO:0046547] (molecular function) Sources: EC:2.1.1.145, RHEA:22200 Also known as: S-adenosyl-L-methionine:(E)-prop-1-ene-1,2,3-tricarboxylate 3'-O-methyltransferase activity Definition: Catalysis of the reaction: S-adenosyl-L-methionine(1+) + trans-aconitate = (E)-2-(methoxycarbonylmethyl)but-2-enedioate + S-adenosyl-L-homocysteine. Relationships: is a type of S-adenosylmethionine-dependent methyltransferase activity [GO:0008757]